{
  "gene": "UniProtKB:Q8IW93",
  "term_id": "UNKNOWN:0003",
  "gene_name": "Rho guanine nucleotide exchange factor 19",
  "term_label": "Unknown cellular component",
  "gene_symbol": "ARHGEF19"
}